{
  "gene_name": "DnaJ homolog subfamily B member 12",
  "term_id": "GO:0030544",
  "gene_symbol": "DNAJB12",
  "term_label": "Hsp70 protein binding",
  "gene": "UniProtKB:Q9NXW2"
}